response to phenylalanine [GO:0080053] (biological process) Subtypes: cellular response to phenylalanine [GO:0071234] Definition: Any process that results in a change in state or activity of a cell or an organism (in terms of movement, secretion, enzyme production, gene expression, etc.) as a result of a phenylalanine stimulus. References: PMID:15889294 Relationships: is a type of response to amino acid [GO:0043200]; is a type of GO:1901698; is a type of GO:1901700